negative regulation of aplanospore formation [GO:0075292] (biological process) Sources: GOC:pamgo_curators Definition: Any process that stops, prevents, or reduces the frequency, rate or extent of aplanospore formation, a process in which a nonmotile, asexual spore is formed within a cell in certain algae and fungi (commonly in the Phycomycetes), the wall of aplanospore is distinct from that of the parent cell. Relationships: is a type of negative regulation of sporangiospore formation [GO:0075288]; is a type of regulation of aplanospore formation [GO:0075290]; negatively regulates GO:0075289